{
  "gene_name": "Tetra-peptide repeat homeobox-like protein",
  "gene": "UniProtKB:Q17RH7",
  "term_id": "UNKNOWN:0001",
  "gene_symbol": "TPRXL",
  "term_label": "Unknown molecular function"
}